Viteagnusin D synthase activity [GO:0062203] (molecular function) References: PMID:29315936 Sources: RHEA:62180 Definition: Catalysis of the reaction: H2O + peregrinol diphosphate = diphosphate + viteagnusin D. Relationships: is a type of carbon-oxygen lyase activity, acting on phosphates [GO:0016838]